{
  "term_id": "GO:0016435",
  "gene_name": "pre-rRNA 2'-O-ribose RNA methyltransferase FTSJ3",
  "term_label": "rRNA (guanine) methyltransferase activity",
  "gene_symbol": "FTSJ3",
  "gene": "UniProtKB:Q8IY81"
}